positive regulation of gluconeogenesis [GO:0045722] (biological process) Definition: Any process that activates or increases the frequency, rate or extent of gluconeogenesis. Sources: GOC:go_curators Also known as: up regulation of gluconeogenesis, up-regulation of gluconeogenesis, upregulation of gluconeogenesis, activation of gluconeogenesis, stimulation of gluconeogenesis Relationships: is_a regulation of gluconeogenesis [GO:0006111]; is a type of positive regulation of biosynthetic process [GO:0009891]; is_a GO:0010907; positively regulates gluconeogenesis [GO:0006094]